{
  "gene_name": "N-acetylaspartate synthetase",
  "gene_symbol": "NAT8L",
  "gene": "UniProtKB:Q8N9F0",
  "term_id": "UNKNOWN:0002",
  "term_label": "Unknown biological process"
}